{
  "gene": "UniProtKB:P13994",
  "gene_name": "Probable splicing factor YJU2B",
  "gene_symbol": "YJU2B",
  "term_label": "Unknown molecular function",
  "term_id": "UNKNOWN:0001"
}